cellular response to amine stimulus [GO:0071418] (biological process) Relationships: is a type of response to amine [GO:0014075]; is_a cellular response to nitrogen compound [GO:1901699] Sources: GOC:mah Subtypes: cellular response to methylamine [GO:0036256], cellular response to amphetamine [GO:0071419], cellular response to hesperadin [GO:0072763], cellular response to methamphetamine hydrochloride [GO:1904314] Definition: Any process that results in a change in state or activity of a cell (in terms of movement, secretion, enzyme production, gene expression, etc.) as a result of an amine stimulus. An amine is a compound formally derived from ammonia by replacing one, two or three hydrogen atoms by hydrocarbyl groups.